{
  "term_id": "GO:0001665",
  "gene_symbol": "ST6GALNAC1",
  "term_label": "alpha-N-acetylgalactosaminide alpha-2,6-sialyltransferase activity",
  "gene": "UniProtKB:Q9NSC7",
  "gene_name": "Alpha-N-acetylgalactosaminide alpha-2,6-sialyltransferase 1"
}